{
  "gene": "UniProtKB:O15520",
  "gene_name": "Fibroblast growth factor 10",
  "term_label": "wound healing",
  "term_id": "GO:0042060",
  "gene_symbol": "FGF10"
}